RNA polymerase III complex [GO:0005666] (cellular component) Relationships: is a type of DNA-directed RNA polymerase complex [GO:0000428]; is a type of nuclear protein-containing complex [GO:0140513] Definition: RNA polymerase III, one of three nuclear DNA-directed RNA polymerases found in all eukaryotes, is a multisubunit complex; typically it produces 5S rRNA, tRNAs and some of the small nuclear RNAs. Two large subunits comprise the most conserved portion including the catalytic site and share similarity with other eukaryotic and bacterial multisubunit RNA polymerases. The remainder of the complex is composed of smaller subunits (generally ten or more), some of which are also found in RNA polymerase I and others of which are also found in RNA polymerases I and II. Although the core is competent to mediate ribonucleic acid synthesis, it requires additional factors to select the appropriate template. Sources: GOC:krc, GOC:mtg_sensu Also known as: DNA-directed RNA polymerase III complex, DNA-directed RNA polymerase III activity